negative regulation of cyclin-dependent protein kinase activity [GO:1904030] (biological process) Also known as: down regulation of cyclin-dependent protein kinase activity, down-regulation of cyclin-dependent protein kinase activity, downregulation of cyclin-dependent protein kinase activity, inhibition of cyclin-dependent protein kinase activity Definition: Any process that stops, prevents or reduces the frequency, rate or extent of cyclin-dependent protein kinase activity. Subtypes: negative regulation of cyclin-dependent protein serine/threonine kinase activity [GO:0045736] References: PMID:22995177 Sources: GOC:TermGenie, GOC:als, GO_REF:0000059 Relationships: is a type of negative regulation of protein kinase activity [GO:0006469]; negatively regulates GO:0097472